liver development [GO:0001889] (biological process) Definition: The process whose specific outcome is the progression of the liver over time, from its formation to the mature structure. The liver is an exocrine gland which secretes bile and functions in metabolism of protein and carbohydrate and fat, synthesizes substances involved in the clotting of the blood, synthesizes vitamin A, detoxifies poisonous substances, stores glycogen, and breaks down worn-out erythrocytes. Sources: GOC:add, ISBN:068340007X Relationships: is a type of gland development [GO:0048732]; is part of hepaticobiliary system development [GO:0061008] Subtypes: liver regeneration [GO:0097421]